{
  "gene_symbol": "BUB1B",
  "term_label": "nucleus",
  "gene": "UniProtKB:O60566",
  "gene_name": "Mitotic checkpoint serine_threonine-protein kinase BUB1 beta",
  "term_id": "GO:0005634"
}